{
  "term_label": "Unknown biological process",
  "gene_symbol": "C7orf31",
  "gene": "UniProtKB:Q8N865",
  "gene_name": "Uncharacterized protein C7orf31",
  "term_id": "UNKNOWN:0002"
}